[2Fe-2S] cluster assembly [GO:0044571] (biological process) Regulation: regulated by regulation of [2Fe-2S] cluster assembly [GO:1900487]; negatively regulated by negative regulation of [2Fe-2S] cluster assembly [GO:1900488]; positively regulated by positive regulation of [2Fe-2S] cluster assembly [GO:1900489] Also known as: 2Fe-2S cluster assembly, [2Fe-2S] cluster biosynthetic process Relationships: is a type of iron-sulfur cluster assembly [GO:0016226] References: PMID:15952888 Sources: GOC:jl, GOC:mengo_curators, GOC:pde, GOC:tt, GOC:vw Definition: The incorporation of two iron atoms and two sulfur atoms into an iron-sulfur cluster.